{
  "gene_name": "Nucleophosmin",
  "gene": "UniProtKB:P06748",
  "term_label": "chromatin remodeling",
  "term_id": "GO:0006338",
  "gene_symbol": "NPM1"
}